{
  "gene_symbol": "FAM181B",
  "term_id": "UNKNOWN:0001",
  "gene_name": "Protein FAM181B",
  "gene": "UniProtKB:A6NEQ2",
  "term_label": "Unknown molecular function"
}